{
  "term_id": "UNKNOWN:0002",
  "gene_symbol": "SUN1",
  "gene": "UniProtKB:O94901",
  "gene_name": "SUN domain-containing protein 1",
  "term_label": "Unknown biological process"
}